{
  "gene_name": "Exportin-1",
  "gene_symbol": "XPO1",
  "term_id": "GO:0005737",
  "term_label": "cytoplasm",
  "gene": "UniProtKB:O14980"
}